polyprenol dehydrogenase (NAD+) activity [GO:0160196] (molecular function) Also known as: polyprenol dehydrogenase activity References: PMID:38821050 Sources: RHEA:80719 Definition: Catalysis of the reaction: a di-trans,poly-cis-polyprenol + NAD+ = a di-trans,poly-cis-polyprenal + NADH + H+. Relationships: is a type of GO:0016628